{
  "gene": "UniProtKB:Q86SX3",
  "gene_name": "Tubulin epsilon and delta complex protein 1",
  "gene_symbol": "TEDC1",
  "term_id": "UNKNOWN:0002",
  "term_label": "Unknown biological process"
}